{
  "term_id": "GO:0006644",
  "gene": "UniProtKB:O14494",
  "gene_symbol": "PLPP1",
  "gene_name": "Phospholipid phosphatase 1",
  "term_label": "phospholipid metabolic process"
}